somatic stem cell population maintenance [GO:0035019] (biological process) Subtypes: mesenchymal stem cell maintenance involved in nephron morphogenesis [GO:0072038], skeletal muscle satellite stem cell maintenance involved in skeletal muscle regeneration [GO:0098731] Relationships: is a type of stem cell population maintenance [GO:0019827] Regulation: regulated by GO:1904672; negatively regulated by negative regulation of somatic stem cell population maintenance [GO:1904673]; positively regulated by GO:1904674 Sources: GOC:bf, ISBN:0582227089 Definition: Any process by which an organism retains a population of somatic stem cells, undifferentiated cells in the embryo or adult which can undergo unlimited division and give rise to cell types of the body other than those of the germ-line.